{
  "gene_symbol": "HNRNPCL4",
  "term_label": "Unknown biological process",
  "gene_name": "Heterogeneous nuclear ribonucleoprotein C-like 4",
  "gene": "UniProtKB:P0DMR1",
  "term_id": "UNKNOWN:0002"
}